{
  "gene": "UniProtKB:Q9GZV9",
  "gene_symbol": "FGF23",
  "gene_name": "Fibroblast growth factor 23",
  "term_label": "type 1 fibroblast growth factor receptor binding",
  "term_id": "GO:0005105"
}